3-methyl-2-oxobutanoate hydroxymethyltransferase activity [GO:0003864] (molecular function) Also known as: 5,10-methylene tetrahydrofolate:alpha-ketoisovalerate hydroxymethyltransferase activity, 5,10-methylenetetrahydrofolate:3-methyl-2-oxobutanoate hydroxymethyltransferase activity, alpha-ketoisovalerate hydroxymethyltransferase activity, dehydropantoate hydroxymethyltransferase activity, ketopantoate hydroxymethyltransferase activity, oxopantoate hydroxymethyltransferase activity Sources: EC:2.1.2.11 Relationships: is a type of hydroxymethyl-, formyl- and related transferase activity [GO:0016742] Definition: Catalysis of the reaction: 5,10-methylenetetrahydrofolate + 3-methyl-2-oxobutanoate = tetrahydrofolate + 2-dehydropantoate.